{
  "term_label": "plasma membrane",
  "term_id": "GO:0005886",
  "gene_symbol": "MYO1G",
  "gene_name": "Unconventional myosin-Ig",
  "gene": "UniProtKB:B0I1T2"
}